{
  "term_id": "UNKNOWN:0002",
  "gene_symbol": "DPH5",
  "gene_name": "Diphthine methyl ester synthase",
  "term_label": "Unknown biological process",
  "gene": "UniProtKB:Q9H2P9"
}